{
  "term_id": "GO:0072558",
  "gene_name": "Caspase-5",
  "term_label": "NLRP1 inflammasome complex",
  "gene": "UniProtKB:P51878",
  "gene_symbol": "CASP5"
}